{
  "gene_symbol": "LINC01546",
  "term_label": "Unknown molecular function",
  "term_id": "UNKNOWN:0001",
  "gene_name": "Putative uncharacterized protein encoded by LINC01546",
  "gene": "UniProtKB:A6NGU7"
}